response to D-galactosamine [GO:1904421] (biological process) Relationships: is a type of response to oxygen-containing compound [GO:1901700] Subtypes: cellular response to D-galactosamine [GO:1904422] References: PMID:12057922 Sources: GOC:TermGenie, GO_REF:0000071 Definition: Any process that results in a change in state or activity of a cell or an organism (in terms of movement, secretion, enzyme production, gene expression, etc.) as a result of a D-galactosamine stimulus.